positive regulation of intestinal cholesterol absorption [GO:0045797] (biological process) Sources: GOC:go_curators Relationships: is a type of GO:0030300; is a type of positive regulation of intestinal lipid absorption [GO:1904731]; positively regulates intestinal cholesterol absorption [GO:0030299] Also known as: up regulation of cholesterol absorption, up-regulation of cholesterol absorption, upregulation of cholesterol absorption, activation of cholesterol absorption, stimulation of cholesterol absorption Definition: Any process that activates or increases the frequency, rate or extent of uptake of cholesterol into the blood by absorption from the intestine.